{
  "term_id": "UNKNOWN:0003",
  "gene_name": "Putative inactive cytochrome P450 2G1",
  "gene": "UniProtKB:Q6ZSU1",
  "term_label": "Unknown cellular component",
  "gene_symbol": "CYP2G1P"
}